{
  "term_id": "UNKNOWN:0003",
  "gene": "UniProtKB:A6NC05",
  "gene_symbol": "C5orf63",
  "gene_name": "Glutaredoxin-like protein C5orf63",
  "term_label": "Unknown cellular component"
}